VEGF-activated neuropilin signaling pathway involved in axon guidance [GO:1902378] (biological process) Definition: Any VEGF-activated neuropilin signaling pathway that is involved in axon guidance. References: PMID:21658587 Sources: GOC:BHF, GOC:TermGenie, GOC:rl Relationships: is a type of VEGF-activated neuropilin signaling pathway [GO:0038190]; BFO_0000050 axon guidance [GO:0007411] Also known as: VEGF-activated neuropilin signaling pathway involved in axon pathfinding, VEGF-Npn-1 signaling involved in axon growth cone guidance, VEGF-Npn-1 signaling involved in axon guidance, VEGF-Npn-1 signaling involved in axon pathfinding, VEGF-activated neuropilin signaling pathway involved in axon growth cone guidance, VEGF-Npn-1 signaling involved in axon chemotaxis, VEGF-activated neuropilin signaling pathway involved in axon chemotaxis, vascular endothelial growth factor-activated neuropilin signaling pathway involved in axon chemotaxis, vascular endothelial growth factor-activated neuropilin signaling pathway involved in axon growth cone guidance, vascular endothelial growth factor-activated neuropilin signaling pathway involved in axon guidance, vascular endothelial growth factor-activated neuropilin signaling pathway involved in axon pathfinding